{
  "term_label": "cytoplasm",
  "gene_name": "Beta-synuclein",
  "gene_symbol": "SNCB",
  "term_id": "GO:0005737",
  "gene": "UniProtKB:Q16143"
}